{
  "term_id": "GO:0000398",
  "gene": "UniProtKB:P51991",
  "gene_name": "Heterogeneous nuclear ribonucleoprotein A3",
  "gene_symbol": "HNRNPA3",
  "term_label": "mRNA splicing, via spliceosome"
}